{
  "term_label": "neuron differentiation",
  "gene_symbol": "WNT11",
  "term_id": "GO:0030182",
  "gene_name": "Protein Wnt-11",
  "gene": "UniProtKB:O96014"
}